mannosyl-oligosaccharide mannosidase activity [GO:0015924] (molecular function) Sources: GOC:ai Definition: Catalysis of the hydrolysis of the terminal alpha-D-mannose residues in oligo-mannose oligosaccharides. Subtypes: mannosyl-oligosaccharide 1,2-alpha-mannosidase activity [GO:0004571], mannosyl-oligosaccharide 1,3-1,6-alpha-mannosidase activity [GO:0004572], GO:0052767, mannosyl-oligosaccharide 1,3-alpha-mannosidase activity [GO:0052768] Relationships: is a type of alpha-mannosidase activity [GO:0004559]